{
  "gene_symbol": "FOXD1",
  "gene_name": "Forkhead box protein D1",
  "gene": "UniProtKB:Q16676",
  "term_id": "GO:0009653",
  "term_label": "anatomical structure morphogenesis"
}